host cell periphery [GO:0044538] (cellular component) Relationships: is a type of GO:0033643 Definition: The part of a cell encompassing the cell cortex, the plasma membrane, and any external encapsulating structures of a host cell. References: PMID:20463076 Sources: GOC:jl